purine deoxyribonucleoside diphosphate catabolic process [GO:0009184] (biological process) Definition: The chemical reactions and pathways resulting in the breakdown of purine deoxyribonucleoside diphosphate, a compound consisting of a purine base linked to a deoxyribose sugar esterified with diphosphate on the sugar. Sources: GOC:go_curators, ISBN:0198506732 Relationships: is_a purine nucleoside diphosphate catabolic process [GO:0009137]; is_a purine deoxyribonucleoside diphosphate metabolic process [GO:0009182]; is a type of deoxyribonucleoside diphosphate catabolic process [GO:0009192] Subtypes: GO:0046057, dGDP catabolic process [GO:0046067] Also known as: purine deoxyribonucleoside diphosphate breakdown, purine deoxyribonucleoside diphosphate catabolism, purine deoxyribonucleoside diphosphate degradation